{
  "gene_name": "Vesicle-associated membrane protein-associated protein A",
  "gene": "UniProtKB:Q9P0L0",
  "term_id": "GO:0043495",
  "term_label": "protein-membrane adaptor activity",
  "gene_symbol": "VAPA"
}